{
  "term_label": "nucleus",
  "gene_symbol": "ZNF665",
  "term_id": "GO:0005634",
  "gene": "UniProtKB:Q9H7R5",
  "gene_name": "Zinc finger protein 665"
}